regulation of RNA polymerase II transcription preinitiation complex assembly [GO:0045898] (biological process) Sources: GOC:go_curators Definition: Any process that modulates the frequency, rate or extent of RNA polymerase II transcriptional preinitiation complex assembly. Also known as: regulation of RNA polymerase II transcriptional pre-initiation complex assembly, regulation of RNA polymerase II transcriptional pre-initiation complex biosynthesis, regulation of RNA polymerase II transcriptional preinitiation complex assembly, regulation of RNA polymerase II transcriptional preinitiation complex formation Relationships: is a type of regulation of protein-containing complex assembly [GO:0043254]; is a type of regulation of transcription initiation by RNA polymerase II [GO:0060260]; regulates GO:0051123 Subtypes: negative regulation of RNA polymerase II transcription preinitiation complex assembly [GO:0017055], positive regulation of RNA polymerase II transcription preinitiation complex assembly [GO:0045899]